positive regulation of macroautophagy [GO:0016239] (biological process) Definition: Any process, such as recognition of nutrient depletion, that activates or increases the rate of macroautophagy to bring cytosolic macromolecules to the vacuole/lysosome for degradation. References: PMID:9412464 Sources: GOC:go_curators Also known as: positive regulation of starvation-induced autophagy, up regulation of macroautophagy, up-regulation of macroautophagy, upregulation of macroautophagy, activation of macroautophagy, stimulation of macroautophagy Relationships: is_a positive regulation of autophagy [GO:0010508]; is a type of GO:0016241; positively regulates macroautophagy [GO:0016236] Subtypes: positive regulation of reticulophagy [GO:0140501], positive regulation of autophagosome maturation [GO:1901098], GO:1901526, GO:1904417, positive regulation of lipophagy [GO:1904504], positive regulation of aggrephagy [GO:1905337], positive regulation of autophagosome assembly [GO:2000786]